{
  "gene": "UniProtKB:Q8N4W9",
  "gene_symbol": "ZNF808",
  "gene_name": "Zinc finger protein 808",
  "term_id": "GO:0000122",
  "term_label": "negative regulation of transcription by RNA polymerase II"
}